{
  "term_label": "plasma membrane",
  "gene_symbol": "SLC4A10",
  "term_id": "GO:0005886",
  "gene_name": "Sodium-driven chloride bicarbonate exchanger",
  "gene": "UniProtKB:Q6U841"
}